negative regulation of RNA metabolic process [GO:0051253] (biological process) Sources: GOC:ai Subtypes: negative regulation of RNA catabolic process [GO:1902369], negative regulation of RNA biosynthetic process [GO:1902679], negative regulation of mRNA metabolic process [GO:1903312], GO:1903324, negative regulation of tRNA metabolic process [GO:1903327], negative regulation of snRNA pseudouridine synthesis [GO:1905357], negative regulation of rRNA processing [GO:2000233], GO:2000629 Definition: Any process that stops, prevents, or reduces the frequency, rate or extent of the chemical reactions and pathways involving RNA. Also known as: down regulation of RNA metabolic process, down-regulation of RNA metabolic process, downregulation of RNA metabolic process, negative regulation of RNA metabolism, inhibition of RNA metabolic process Relationships: is a type of GO:0010605; is a type of negative regulation of nucleobase-containing compound metabolic process [GO:0045934]; is a type of regulation of RNA metabolic process [GO:0051252]; negatively regulates GO:0016070